{
  "term_id": "GO:0045727",
  "gene_name": "Fragile X messenger ribonucleoprotein 1",
  "gene": "UniProtKB:Q06787",
  "gene_symbol": "FMR1",
  "term_label": "positive regulation of translation"
}